{
  "term_id": "GO:0045944",
  "gene_name": "Cyclin-C",
  "gene_symbol": "CCNC",
  "gene": "UniProtKB:P24863",
  "term_label": "positive regulation of transcription by RNA polymerase II"
}